{
  "term_id": "UNKNOWN:0001",
  "gene_symbol": "RIPPLY3",
  "gene_name": "Protein ripply3",
  "term_label": "Unknown molecular function",
  "gene": "UniProtKB:P57055"
}